{
  "gene_symbol": "SLIT3",
  "term_id": "GO:0050919",
  "gene_name": "Slit homolog 3 protein",
  "term_label": "negative chemotaxis",
  "gene": "UniProtKB:O75094"
}